alpha-ketoglutarate-dependent xanthine dioxygenase activity [GO:0097641] (molecular function) Also known as: 2-oxoglutarate-dependent xanthine dioxygenase activity, alpha-ketoglutarate- and Fe(II)-dependent xanthine dioxygenase activity, alpha-ketoglutarate- and Fe(II)-dependent xanthine hydroxylase activity Definition: Catalysis of the reaction: 2-oxoglutarate (alpha-ketoglutarate) + O2 + xanthine = CO2 + succinate + urate. Relationships: is a type of GO:0051213 References: PMID:15948966, PMID:17429948 Sources: GOC:vw, RHEA:43120